regulation of pancreatic trypsinogen secretion [GO:1904242] (BP) Also known as: regulation of pancreatic trypsinogen release Subtypes: negative regulation of pancreatic trypsinogen secretion [GO:1904243], positive regulation of pancreatic trypsinogen secretion [GO:1904244] Definition: Any process that modulates the frequency, rate or extent of pancreatic trypsinogen secretion. References: PMID:12771515 Sources: GOC:TermGenie, GO_REF:0000058 Relationships: is a type of regulation of protein secretion [GO:0050708]; regulates pancreatic trypsinogen secretion [GO:1990747]